{
  "term_label": "Unknown biological process",
  "gene_name": "Coiled-coil domain-containing protein 159",
  "gene_symbol": "CCDC159",
  "gene": "UniProtKB:P0C7I6",
  "term_id": "UNKNOWN:0002"
}